{
  "gene_name": "Syntabulin",
  "term_label": "axonal transport of mitochondrion",
  "gene_symbol": "SYBU",
  "gene": "UniProtKB:Q9NX95",
  "term_id": "GO:0019896"
}